{
  "term_id": "GO:0005737",
  "term_label": "cytoplasm",
  "gene_symbol": "HIPK3",
  "gene_name": "Homeodomain-interacting protein kinase 3",
  "gene": "UniProtKB:Q9H422"
}